{
  "term_label": "clathrin-coated pit",
  "gene_name": "Disabled homolog 2",
  "term_id": "GO:0005905",
  "gene": "UniProtKB:P98082",
  "gene_symbol": "DAB2"
}